larval salivary gland boundary specification [GO:0007433] (biological process) References: PMID:11598957 Sources: GOC:tb Regulation: regulated by regulation of larval salivary gland boundary specification [GO:0045708]; negatively regulated by negative regulation of larval salivary gland boundary specification [GO:0045710]; positively regulated by GO:0045712 Definition: Determination in a larval organism of where the salivary gland forms, the total number of salivary gland cells and how many cells are allocated to each of the specialised cell types within the salivary gland. Relationships: is a type of salivary gland boundary specification [GO:0007432]; is part of instar larval development [GO:0002168] Also known as: larval salivary gland determination